histone H3R2 demethylase activity [GO:0033746] (molecular function) Definition: Catalysis of the removal of the methyl group from a modified arginine residue at position 2 of the histone H3 protein. This is a dioxygenase reaction that is dependent on Fe(II) and 2-oxoglutarate. Also known as: histone H3-R2 demethylase activity, histone H3-methyl-arginine-2 demethylase activity, histone H3R2me demethylase activity, histone demethylase activity (H3-R2 specific) Note: Comment: Note that the residue position corresponds to the canonical human H3 histone (UniProtKB:P84243); this residue is conserved across all eukaryotes. Residue 1 is the first residue following removal of the initiating Methionine (Met). Note that each histone is encoded by multiple genes, and sequences may vary across different genes within an organism. Relationships: is a type of GO:0016706; is a type of GO:0141052 References: PMID:17947579, PMID:22483719, PMID:29233856